cinnamic acid ester biosynthetic process [GO:0009802] (biological process) Also known as: cinnamic acid ester anabolism, cinnamic acid ester biosynthesis, cinnamic acid ester formation, cinnamic acid ester synthesis, cinnamylic acid ester biosynthesis, cinnamylic acid ester biosynthetic process, phenylacrylic acid ester biosynthesis, phenylacrylic acid ester biosynthetic process Subtypes: GO:0090431 Relationships: is a type of GO:0009699; is a type of cinnamic acid ester metabolic process [GO:0009801]; is a type of olefinic compound biosynthetic process [GO:0120255]; is part of cinnamic acid metabolic process [GO:0009803] Definition: The chemical reactions and pathways resulting in the formation of ester derivatives of cinnamic acid, phenylpropenoic acid. Sources: GOC:jl